{
  "gene": "UniProtKB:Q6V1P9",
  "gene_name": "Protocadherin-23",
  "gene_symbol": "DCHS2",
  "term_label": "adherens junction",
  "term_id": "GO:0005912"
}